phytochelatin metabolic process [GO:0046937] (biological process) Definition: The chemical reactions and pathways involving phytochelatins, any of a group of peptides that bind metals (Cd, Zn, Cu, Pb, Hg) in thiolate coordination complexes. The structure is of the type (gamma-glutamyl-cysteinyl)n-glycine, where n is 2 to 11. Also known as: phytochelatin metabolism, cadystin metabolic process, cadystin metabolism Relationships: is a type of amide metabolic process [GO:0043603]; is a type of primary metabolic process [GO:0044238] Sources: ISBN:0198506732 Subtypes: phytochelatin biosynthetic process [GO:0046938], phytochelatin-metal complex formation [GO:0090423], phytochelatin-metal-sulfur complex formation [GO:0090424]